{
  "gene_name": "Putative protein SPATA31F2P",
  "gene": "UniProtKB:Q63HN1",
  "gene_symbol": "SPATA31F2P",
  "term_label": "Unknown molecular function",
  "term_id": "UNKNOWN:0001"
}